negative regulation of emericellin biosynthetic process [GO:1900835] (biological process) Sources: GOC:TermGenie, GOC:di Definition: Any process that stops, prevents or reduces the frequency, rate or extent of emericellin biosynthetic process. Relationships: is a type of GO:1900184; is a type of negative regulation of secondary metabolite biosynthetic process [GO:1900377]; is a type of regulation of emericellin biosynthetic process [GO:1900834]; negatively regulates emericellin biosynthetic process [GO:1900766] Also known as: down regulation of emericellin biosynthetic process, down-regulation of emericellin biosynthetic process, downregulation of emericellin biosynthetic process